{
  "gene_name": "Neuronal acetylcholine receptor subunit alpha-6",
  "gene": "UniProtKB:Q15825",
  "term_id": "GO:0007271",
  "gene_symbol": "CHRNA6",
  "term_label": "synaptic transmission, cholinergic"
}